{
  "gene_symbol": "CABLES2",
  "term_label": "Unknown cellular component",
  "gene_name": "CDK5 and ABL1 enzyme substrate 2",
  "term_id": "UNKNOWN:0003",
  "gene": "UniProtKB:Q9BTV7"
}